{
  "gene_symbol": "FOXL3",
  "term_label": "cell differentiation",
  "term_id": "GO:0030154",
  "gene_name": "Forkhead box protein L3",
  "gene": "UniProtKB:A0A1W2PRP0"
}